{
  "gene_name": "Transcription factor SOX-21",
  "term_id": "GO:0000978",
  "term_label": "RNA polymerase II cis-regulatory region sequence-specific DNA binding",
  "gene_symbol": "SOX21",
  "gene": "UniProtKB:Q9Y651"
}